{
  "term_id": "UNKNOWN:0002",
  "gene_name": "Platelet-derived growth factor receptor-like protein",
  "gene": "UniProtKB:Q15198",
  "gene_symbol": "PDGFRL",
  "term_label": "Unknown biological process"
}